{
  "gene_name": "Ectonucleoside triphosphate diphosphohydrolase 3",
  "term_id": "GO:0009134",
  "term_label": "nucleoside diphosphate catabolic process",
  "gene_symbol": "ENTPD3",
  "gene": "UniProtKB:O75355"
}